{
  "gene": "UniProtKB:Q9ULZ0",
  "gene_name": "TP53-target gene 3 protein",
  "term_id": "UNKNOWN:0001",
  "term_label": "Unknown molecular function",
  "gene_symbol": "TP53TG3F"
}